{
  "term_id": "GO:2001235",
  "gene_symbol": "TRIM39",
  "gene_name": "E3 ubiquitin-protein ligase TRIM39",
  "term_label": "positive regulation of apoptotic signaling pathway",
  "gene": "UniProtKB:Q9HCM9"
}